myosin XI complex [GO:0031481] (cellular component) References: PMID:22973289, PMID:29307817 Definition: A myosin complex containing a dimer of class XI myosin heavy chains and associated light chains. Myosin XI heavy chain sizes are similar in molecular structure to the class V myosins with 5 to 6 IQ motifs and tail regions with predicted coiled coil domains (forming dimeric molecules) and large C-terminal regions. Relationships: is a type of unconventional myosin complex [GO:0016461]